{
  "gene_symbol": "REPS2",
  "term_label": "cytoplasm",
  "gene": "UniProtKB:Q8NFH8",
  "gene_name": "RalBP1-associated Eps domain-containing protein 2",
  "term_id": "GO:0005737"
}